{
  "term_id": "GO:0005886",
  "gene": "UniProtKB:P61586",
  "gene_name": "Transforming protein RhoA",
  "gene_symbol": "RHOA",
  "term_label": "plasma membrane"
}